{
  "gene": "UniProtKB:Q8IWA6",
  "gene_name": "Coiled-coil domain-containing protein 60",
  "term_label": "Unknown molecular function",
  "term_id": "UNKNOWN:0001",
  "gene_symbol": "CCDC60"
}